17-beta-hydroxysteroid dehydrogenase (NAD+) activity [GO:0044594] (molecular function) Subtypes: testosterone dehydrogenase (NAD+) activity [GO:0047035] Definition: Catalysis of the reaction: a 17-beta-hydroxysteroid + NAD+ = a 17-oxosteroid + NADH + H+. Relationships: is a type of steroid dehydrogenase activity, acting on the CH-OH group of donors, NAD or NADP as acceptor [GO:0033764] References: PMID:17074428 Sources: RHEA:81599